{
  "term_id": "GO:0042393",
  "gene": "UniProtKB:O14647",
  "gene_symbol": "CHD2",
  "term_label": "histone binding",
  "gene_name": "Chromodomain-helicase-DNA-binding protein 2"
}